{
  "gene_name": "Killer cell immunoglobulin-like receptor, three Ig domains pseudogene 1",
  "gene_symbol": "KIR3DP1",
  "term_label": "plasma membrane",
  "term_id": "GO:0005886",
  "gene": "UniProtKB:A0A0G2JN01"
}